{
  "gene_name": "Achaete-scute homolog 2",
  "gene_symbol": "ASCL2",
  "gene": "UniProtKB:Q99929",
  "term_label": "positive regulation of transcription by RNA polymerase II",
  "term_id": "GO:0045944"
}